{
  "gene_symbol": "TMEM120A",
  "term_id": "GO:0045444",
  "gene_name": "Ion channel TACAN",
  "gene": "UniProtKB:Q9BXJ8",
  "term_label": "fat cell differentiation"
}